{
  "gene_symbol": "ZSCAN26",
  "gene": "UniProtKB:Q16670",
  "gene_name": "Zinc finger and SCAN domain-containing protein 26",
  "term_id": "GO:0000978",
  "term_label": "RNA polymerase II cis-regulatory region sequence-specific DNA binding"
}